collagen network [GO:0098645] (cellular component) Subtypes: interstitial hexagonal collagen network [GO:0098646], chicken-wire-like collagen network [GO:0140154], hexagonal collagen network of basement membrane [GO:0140155] References: PMID:21421911 Sources: GOC:dos Relationships: is_a complex of collagen trimers [GO:0098644] Definition: A supramolecular complex that consists of collagen triple helices associated to form a network.